{
  "term_label": "extracellular space",
  "gene_name": "Bone morphogenetic protein 5",
  "gene": "UniProtKB:P22003",
  "gene_symbol": "BMP5",
  "term_id": "GO:0005615"
}